tracheal pit formation in open tracheal system [GO:0035202] (BP) Relationships: is a type of anatomical structure formation involved in morphogenesis [GO:0048646]; BFO_0000050 open tracheal system development [GO:0007424] Also known as: tracheal sac formation, tracheal placode invagination Definition: Formation of the tracheal pits, the first tube-like structures to form in the open tracheal system. Once cells are determined to their tracheal cell fate, the tracheal pits arise by invagination of each ectodermal cluster of tracheal placode cells, between 5 and 7 hours after egg laying. An example of this is found in Drosophila melanogaster. References: PMID:11063940, PMID:11992723, PMID:14570584 Sources: GOC:mtg_sensu